{
  "term_label": "detection of mechanical stimulus",
  "gene": "UniProtKB:Q92508",
  "term_id": "GO:0050982",
  "gene_symbol": "PIEZO1",
  "gene_name": "Piezo-type mechanosensitive ion channel component 1"
}